{
  "term_label": "sequence-specific DNA binding",
  "term_id": "GO:0043565",
  "gene_symbol": "CBFB",
  "gene": "UniProtKB:Q13951",
  "gene_name": "Core-binding factor subunit beta"
}